maintenance of protein location in membrane [GO:0072658] (biological process) Subtypes: GO:0072660 Sources: GOC:mah Relationships: is a type of maintenance of protein location in cell [GO:0032507]; is part of protein localization to membrane [GO:0072657] Definition: Any process in which a protein is maintained in a specific location in a membrane, and is prevented from moving elsewhere.